{
  "gene": "UniProtKB:O95999",
  "term_id": "GO:2001238",
  "gene_symbol": "BCL10",
  "term_label": "positive regulation of extrinsic apoptotic signaling pathway",
  "gene_name": "B-cell lymphoma_leukemia 10"
}